{
  "term_id": "GO:0005634",
  "gene": "UniProtKB:Q00403",
  "gene_name": "Transcription initiation factor IIB",
  "term_label": "nucleus",
  "gene_symbol": "GTF2B"
}